{
  "gene_symbol": "MAP3K1",
  "term_label": "protein serine/threonine kinase activity",
  "gene": "UniProtKB:Q13233",
  "term_id": "GO:0004674",
  "gene_name": "Mitogen-activated protein kinase kinase kinase 1"
}